regulation of gastro-intestinal system smooth muscle contraction [GO:1904304] (biological process) Relationships: is a type of regulation of smooth muscle contraction [GO:0006940]; RO_0002211 gastro-intestinal system smooth muscle contraction [GO:0014831] Definition: Any process that modulates the frequency, rate or extent of gastro-intestinal system smooth muscle contraction. References: PMID:10821044 Sources: GOC:TermGenie, GO_REF:0000058 Subtypes: regulation of stomach fundus smooth muscle contraction [GO:0120068], regulation of pyloric antrum smooth muscle contraction [GO:0120071], GO:1904305, GO:1904306, GO:1904341, GO:1904347